positive regulation of pseudopodium assembly [GO:0031274] (biological process) Also known as: activation of pseudopodium formation, stimulation of pseudopodium formation, positive regulation of pseudopodium formation, up regulation of pseudopodium formation, up-regulation of pseudopodium formation, upregulation of pseudopodium formation Relationships: is a type of GO:0031272; is a type of positive regulation of plasma membrane bounded cell projection assembly [GO:0120034]; positively regulates pseudopodium assembly [GO:0031269] Sources: GOC:pg Definition: Any process that activates or increases the frequency, rate or extent of the assembly of pseudopodia.